enhanceosome [GO:0034206] (cellular component) Relationships: is a type of protein-DNA complex [GO:0032993] Definition: A protein-DNA complex formed by the association of a distinct set of general and specific transcription factors with a region of enhancer DNA. The cooperative assembly of an enhanceosome confers specificity of transcriptional regulation. References: PMID:11250145, PMID:17574024